pyruvate kinase activity [GO:0004743] (molecular function) Also known as: ATP:pyruvate 2-O-phosphotransferase activity, phosphoenol transphosphorylase activity, phosphoenolpyruvate kinase activity Regulation: regulated by GO:1903302 Relationships: is_a phosphotransferase activity, alcohol group as acceptor [GO:0016773]; is part of glycolytic process [GO:0006096] Sources: RHEA:18157 Definition: Catalysis of the reaction: ADP + H+ + phosphoenolpyruvate = ATP + pyruvate.